{
  "term_label": "plasma membrane",
  "gene": "UniProtKB:Q9GZU1",
  "gene_name": "Mucolipin-1",
  "term_id": "GO:0005886",
  "gene_symbol": "MCOLN1"
}